{
  "term_id": "UNKNOWN:0002",
  "term_label": "Unknown biological process",
  "gene_name": "Low-density lipoprotein receptor-related protein 5-like protein",
  "gene_symbol": "LRP5L",
  "gene": "UniProtKB:A4QPB2"
}